{
  "term_label": "Unknown molecular function",
  "gene_name": "Citron Rho-interacting kinase",
  "gene_symbol": "CIT",
  "term_id": "UNKNOWN:0001",
  "gene": "UniProtKB:O14578"
}